Wnt signalosome assembly [GO:1904887] (BP) Also known as: LRP5/6 signalosome assembly, LRP5/6 signalosome formation, Wnt signalosome complex assembly, Wnt signalosome complex formation, Wnt signalosome formation, Wnt-LRP5/6 signalosome assembly, Wnt-LRP5/6 signalosome formation, LRP6 signalosome assembly, LRP6 signalosome formation Relationships: is a type of protein-containing complex assembly [GO:0065003] References: PMID:22899650 Sources: GOC:PARL, GOC:TermGenie, GOC:bf, GO_REF:0000079 Definition: The aggregation, arrangement and bonding together of a set of components to form a Wnt signalosome.